{
  "term_id": "GO:0035091",
  "gene": "UniProtKB:Q92543",
  "gene_symbol": "SNX19",
  "term_label": "phosphatidylinositol binding",
  "gene_name": "Sorting nexin-19"
}